{
  "gene_symbol": "NR1I3",
  "term_label": "intracellular receptor signaling pathway",
  "gene": "UniProtKB:Q14994",
  "gene_name": "Nuclear receptor subfamily 1 group I member 3",
  "term_id": "GO:0030522"
}